{
  "gene_symbol": "POM121C",
  "gene": "UniProtKB:A8CG34",
  "term_label": "protein import into nucleus",
  "gene_name": "Nuclear envelope pore membrane protein POM 121C",
  "term_id": "GO:0006606"
}